sensory perception of light stimulus [GO:0050953] (biological process) Subtypes: visual perception [GO:0007601] Sources: GOC:ai Relationships: is a type of sensory perception [GO:0007600] Definition: The series of events required for an organism to receive a sensory light stimulus, convert it to a molecular signal, and recognize and characterize the signal. This is a neurological process.